{
  "gene_name": "Carbohydrate sulfotransferase 2",
  "gene_symbol": "CHST2",
  "term_label": "N-acetylglucosamine 6-O-sulfotransferase activity",
  "term_id": "GO:0001517",
  "gene": "UniProtKB:Q9Y4C5"
}